{
  "gene_symbol": "HLA-A",
  "term_id": "GO:0005102",
  "gene": "UniProtKB:P04439",
  "term_label": "signaling receptor binding",
  "gene_name": "HLA class I histocompatibility antigen, A alpha chain"
}